{
  "gene": "UniProtKB:P08235",
  "gene_symbol": "NR3C2",
  "term_id": "GO:0030518",
  "term_label": "nuclear receptor-mediated steroid hormone signaling pathway",
  "gene_name": "Mineralocorticoid receptor"
}